{
  "term_id": "GO:0007034",
  "gene": "UniProtKB:P86791",
  "gene_symbol": "CCZ1",
  "gene_name": "Vacuolar fusion protein CCZ1 homolog",
  "term_label": "vacuolar transport"
}